{
  "gene": "UniProtKB:O95156",
  "term_label": "Unknown biological process",
  "term_id": "UNKNOWN:0002",
  "gene_symbol": "NXPH2",
  "gene_name": "Neurexophilin-2"
}